{
  "gene_symbol": "PPARA",
  "gene_name": "Peroxisome proliferator-activated receptor alpha",
  "term_label": "nuclear receptor activity",
  "gene": "UniProtKB:Q07869",
  "term_id": "GO:0004879"
}